{
  "term_id": "GO:0015389",
  "gene": "UniProtKB:O00337",
  "gene_symbol": "SLC28A1",
  "term_label": "pyrimidine- and adenosine-specific:sodium symporter activity",
  "gene_name": "Sodium_nucleoside cotransporter 1"
}